cell surface toll-like receptor signaling pathway [GO:0140895] (biological process) Definition: The series of molecular signals initiated by a ligand binding to a cell surface pattern recognition receptor (PRR) of the toll-like family. References: PMID:15199967 Sources: GOC:add, GOC:ar, ISBN:0781735149 Also known as: cell surface TLR signaling pathway Relationships: is a type of cell surface pattern recognition receptor signaling pathway [GO:0002752] Subtypes: toll-like receptor 2 signaling pathway [GO:0034134], toll-like receptor 4 signaling pathway [GO:0034142], GO:0034146, toll-like receptor 6 signaling pathway [GO:0034150], toll-like receptor 10 signaling pathway [GO:0034166], GO:0035681